{
  "gene_symbol": "CCDC42",
  "term_id": "UNKNOWN:0003",
  "gene_name": "Coiled-coil domain-containing protein 42",
  "gene": "UniProtKB:Q96M95",
  "term_label": "Unknown cellular component"
}